{
  "gene_symbol": "PRICKLE3",
  "gene_name": "Prickle planar cell polarity protein 3",
  "gene": "UniProtKB:O43900",
  "term_label": "Unknown biological process",
  "term_id": "UNKNOWN:0002"
}